{
  "gene_symbol": "POLD3",
  "gene_name": "DNA polymerase delta subunit 3",
  "term_label": "nucleotide-excision repair, DNA gap filling",
  "gene": "UniProtKB:Q15054",
  "term_id": "GO:0006297"
}